{
  "gene_symbol": "PRICKLE3",
  "gene": "UniProtKB:O43900",
  "term_id": "UNKNOWN:0001",
  "gene_name": "Prickle planar cell polarity protein 3",
  "term_label": "Unknown molecular function"
}